{
  "gene_name": "GTPase NRas",
  "term_label": "plasma membrane",
  "gene_symbol": "NRAS",
  "gene": "UniProtKB:P01111",
  "term_id": "GO:0005886"
}